xanthine DNA N-glycosylase activity [GO:0097508] (molecular function) Definition: DNA N-glycosylase activity acting on deaminated guanine (xanthine). Also known as: xanthine-DNA glycosylase activity Relationships: is a type of GO:0097506 References: PMID:18789404 Sources: GOC:al